{
  "gene": "UniProtKB:P0DSO2",
  "term_label": "Unknown biological process",
  "gene_symbol": "SCYGR9",
  "gene_name": "Small cysteine and glycine repeat-containing protein 9",
  "term_id": "UNKNOWN:0002"
}